{
  "gene_name": "F-box only protein 30",
  "term_label": "Unknown cellular component",
  "gene": "UniProtKB:Q8TB52",
  "gene_symbol": "FBXO30",
  "term_id": "UNKNOWN:0003"
}